{
  "gene_symbol": "TRIM10",
  "term_label": "ubiquitin protein ligase activity",
  "gene": "UniProtKB:Q9UDY6",
  "gene_name": "Tripartite motif-containing protein 10",
  "term_id": "GO:0061630"
}